{
  "gene_name": "Muscarinic acetylcholine receptor M3",
  "term_id": "GO:0007197",
  "term_label": "adenylate cyclase-inhibiting G protein-coupled acetylcholine receptor signaling pathway",
  "gene_symbol": "CHRM3",
  "gene": "UniProtKB:P20309"
}